ruffle membrane [GO:0032587] (cellular component) Definition: The portion of the plasma membrane surrounding a ruffle. Sources: GOC:mah Also known as: membrane ruffle Relationships: is a type of cell projection membrane [GO:0031253]; is a type of GO:0031256; is part of ruffle [GO:0001726]